{
  "term_id": "GO:0050829",
  "gene_symbol": "DEFA6",
  "term_label": "defense response to Gram-negative bacterium",
  "gene_name": "Defensin-6",
  "gene": "UniProtKB:Q01524"
}